U4 snRNP [GO:0005687] (cellular component) Sources: GOC:krc, GOC:mah, ISBN:0879695897 Definition: A ribonucleoprotein complex that contains small nuclear RNA U4, a heptameric ring of Sm proteins, as well as several proteins that are unique to the U4 snRNP, most of which remain associated with the U4 snRNA both while the U4 snRNP is free or assembled into the U4/U6 snRNP or into a series of spliceosomal complexes. Also known as: snRNP U4 Relationships: is a type of spliceosomal snRNP complex [GO:0097525]